arginine decarboxylase activity [GO:0008792] (molecular function) Also known as: L-arginine carboxy-lyase (agmatine-forming), L-arginine carboxy-lyase activity, SpeA Sources: EC:4.1.1.19, RHEA:17641 Definition: Catalysis of the reaction: L-arginine + H+ = agmatine + CO2. Relationships: is a type of carboxy-lyase activity [GO:0016831]